{
  "gene_name": "Phospholipid-transporting ATPase ID",
  "gene": "UniProtKB:P98198",
  "term_id": "GO:0005886",
  "gene_symbol": "ATP8B2",
  "term_label": "plasma membrane"
}